{
  "term_id": "GO:0005634",
  "gene_name": "Fidgetin",
  "term_label": "nucleus",
  "gene": "UniProtKB:Q5HY92",
  "gene_symbol": "FIGN"
}